neuroblast proliferation [GO:0007405] (biological process) Relationships: is a type of GO:0061351; is part of generation of neurons [GO:0048699] Regulation: RO_0002213 by positive regulation of neuroblast proliferation [GO:0002052]; negatively regulated by GO:0007406; regulated by GO:1902692 Sources: GOC:ai, GOC:mtg_sensu, GOC:sart Definition: The expansion of a neuroblast population by cell division. A neuroblast is any cell that will divide and give rise to a neuron.